NAD+-histone H2BE2 glutamate ADP-ribosyltransferase activity [GO:0140844] (molecular function) Also known as: NAD+-histone H2B-E2 glutamate ADP-ribosyltransferase activity, NAD+-histone-glutamate ADP-ribosyltransferase activity (H2B-E2 specific) Definition: Catalysis of the transfer of ADP-ribose groups to the glutamate-2 residue of the N-terminal tail of histone H2B (or an equivalent residue). Note: Note that the residue position corresponds to the canonical human H2B histone (UniProtKB:P62807); the N-terminus of histone H2B is divergent across eukaryotes; make sure that the paper clearly references the human protein for the position of this modification to use this term. Corresponds to histone H2BE18  in Dictyostelium (PMID:28252050). Residue 1 is the first residue following removal of the initiating Methionine (Met). Note that each histone is encoded by multiple genes, and sequences may vary across different genes within an organism. Relationships: is a type of NAD+-protein-glutamate ADP-ribosyltransferase activity [GO:0140807] References: PMID:27530147